negative regulation of cortisol biosynthetic process [GO:2000065] (biological process) Sources: GOC:obol, GOC:yaf Also known as: negative regulation of cortisol biosynthesis, negative regulation of cortisol formation, negative regulation of cortisol synthesis, negative regulation of cortisol anabolism Definition: Any process that stops, prevents, or reduces the frequency, rate or extent of cortisol biosynthetic process. Relationships: is a type of negative regulation of glucocorticoid biosynthetic process [GO:0031947]; is a type of GO:1902931; is a type of regulation of cortisol biosynthetic process [GO:2000064]; RO_0002212 cortisol biosynthetic process [GO:0034651]